regulation of membrane depolarization during cardiac muscle cell action potential [GO:1900825] (BP) Subtypes: negative regulation of membrane depolarization during cardiac muscle cell action potential [GO:1900826], positive regulation of membrane depolarization during cardiac muscle cell action potential [GO:1900827], regulation of membrane depolarization during AV node cell action potential [GO:1905027] Sources: GOC:BHF, GOC:TermGenie, GOC:mtg_cardiac_conduct_nov11 Definition: Any process that modulates the frequency, rate or extent of membrane depolarization during a cardiac muscle cell action potential. Relationships: is a type of GO:0098902; regulates membrane depolarization during cardiac muscle cell action potential [GO:0086012]